{
  "gene_symbol": "MOV10L1",
  "gene": "UniProtKB:Q9BXT6",
  "term_id": "GO:0003723",
  "term_label": "RNA binding",
  "gene_name": "RNA helicase Mov10l1"
}